{
  "gene_symbol": "NUF2",
  "term_id": "GO:0051315",
  "gene_name": "Kinetochore protein Nuf2",
  "term_label": "attachment of mitotic spindle microtubules to kinetochore",
  "gene": "UniProtKB:Q9BZD4"
}